{
  "gene_name": "Probable inactive tRNA-specific adenosine deaminase-like protein 3",
  "term_id": "UNKNOWN:0002",
  "term_label": "Unknown biological process",
  "gene": "UniProtKB:Q96EY9",
  "gene_symbol": "ADAT3"
}